{
  "gene_symbol": "CR1",
  "term_id": "UNKNOWN:0001",
  "gene": "UniProtKB:P17927",
  "term_label": "Unknown molecular function",
  "gene_name": "Complement receptor type 1"
}